{
  "gene_name": "RING finger protein 37",
  "gene_symbol": "UBOX5",
  "term_id": "GO:0000209",
  "term_label": "protein polyubiquitination",
  "gene": "UniProtKB:O94941"
}